{
  "gene_name": "Kelch repeat and BTB domain-containing protein 13",
  "gene": "UniProtKB:C9JR72",
  "term_id": "UNKNOWN:0001",
  "gene_symbol": "KBTBD13",
  "term_label": "Unknown molecular function"
}